erythromycin 3''-o-methyltransferase activity [GO:0102307] (molecular function) Definition: Catalysis of the reaction: erythromycin C + S-adenosyl-L-methionine = erythromycin A + H+ + S-adenosyl-L-homocysteine. Also converts erythromycin D into erythromycin B. Relationships: is a type of methyltransferase activity [GO:0008168] Sources: EC:2.1.1.254 Also known as: erythromycin C 3''-o-methyltransferase activity, erythromycin D 3''-o-methyltransferase activity